{
  "term_label": "Unknown molecular function",
  "gene_name": "Cilia- and flagella-associated protein 43",
  "gene": "UniProtKB:Q8NDM7",
  "term_id": "UNKNOWN:0001",
  "gene_symbol": "CFAP43"
}